triokinase activity [GO:0050354] (molecular function) Sources: EC:2.7.1.28, RHEA:13941 Relationships: is a type of kinase activity [GO:0016301]; is a type of phosphotransferase activity, alcohol group as acceptor [GO:0016773] Also known as: ATP:D-glyceraldehyde 3-phosphotransferase activity, D-triokinase activity, trio triose kinase (phosphorylating), triose kinase activity Definition: Catalysis of the reaction: D-glyceraldehyde + ATP = D-glyceraldehyde 3-phosphate + ADP + 2 H+.